citrulline biosynthetic process [GO:0019240] (biological process) Regulation: regulated by GO:1903248; RO_0002212 by negative regulation of citrulline biosynthetic process [GO:1903249]; positively regulated by GO:1903250 Sources: ISBN:0198506732 Relationships: is a type of citrulline metabolic process [GO:0000052]; is a type of non-proteinogenic amino acid biosynthetic process [GO:0170043]; is a type of alpha-amino acid biosynthetic process [GO:1901607] Definition: The chemical reactions and pathways resulting in the formation of citrulline, N5-carbamoyl-L-ornithine, an alpha amino acid not found in proteins. Also known as: citrulline anabolism, citrulline biosynthesis, citrulline formation, citrulline synthesis